regulation of cell-matrix adhesion [GO:0001952] (biological process) Subtypes: negative regulation of cell-matrix adhesion [GO:0001953], positive regulation of cell-matrix adhesion [GO:0001954], regulation of focal adhesion assembly [GO:0051893], regulation of endothelial cell-matrix adhesion [GO:1904904], regulation of smooth muscle cell-matrix adhesion [GO:2000097] Definition: Any process that modulates the frequency, rate or extent of attachment of a cell to the extracellular matrix. Relationships: is a type of regulation of cell-substrate adhesion [GO:0010810]; regulates cell-matrix adhesion [GO:0007160] Sources: GOC:hjd